positive regulation of Fc-gamma receptor signaling pathway involved in phagocytosis [GO:1905451] (biological process) Relationships: is a type of positive regulation of immune effector process [GO:0002699]; is a type of positive regulation of phagocytosis [GO:0050766]; is a type of positive regulation of Fc receptor mediated stimulatory signaling pathway [GO:0060369]; is a type of regulation of Fc-gamma receptor signaling pathway involved in phagocytosis [GO:1905449]; positively regulates Fc-gamma receptor signaling pathway involved in phagocytosis [GO:0038096] References: PMID:18832707 Sources: GOC:TermGenie, GO_REF:0000058 Also known as: positive regulation of Fc gamma receptor-dependent phagocytosis, positive regulation of Fc-gamma receptor signalling pathway involved in phagocytosis, positive regulation of Fcgamma receptor-mediated phagocytosis, positive regulation of IgG-mediated phagocytosis, up regulation of Fc gamma receptor-dependent phagocytosis, up regulation of Fc-gamma receptor signaling pathway involved in phagocytosis, up regulation of Fc-gamma receptor signalling pathway involved in phagocytosis, up regulation of Fcgamma receptor-mediated phagocytosis, up regulation of IgG-mediated phagocytosis, up-regulation of Fc gamma receptor-dependent phagocytosis, up-regulation of Fc-gamma receptor signaling pathway involved in phagocytosis, up-regulation of Fc-gamma receptor signalling pathway involved in phagocytosis, up-regulation of Fcgamma receptor-mediated phagocytosis, up-regulation of IgG-mediated phagocytosis, upregulation of Fc gamma receptor-dependent phagocytosis, upregulation of Fc-gamma receptor signaling pathway involved in phagocytosis, upregulation of Fc-gamma receptor signalling pathway involved in phagocytosis, upregulation of Fcgamma receptor-mediated phagocytosis, upregulation of IgG-mediated phagocytosis, activation of Fc gamma receptor-dependent phagocytosis, activation of Fc-gamma receptor signaling pathway involved in phagocytosis, activation of Fc-gamma receptor signalling pathway involved in phagocytosis, activation of Fcgamma receptor-mediated phagocytosis, activation of IgG-mediated phagocytosis Definition: Any process that activates or increases the frequency, rate or extent of Fc-gamma receptor signaling pathway involved in phagocytosis.